elastin catabolic process [GO:0060309] (biological process) Regulation: RO_0002211 by GO:0060310; negatively regulated by negative regulation of elastin catabolic process [GO:0060311]; positively regulated by GO:0110015 Relationships: is a type of glycoprotein catabolic process [GO:0006516]; is a type of elastin metabolic process [GO:0051541] Definition: The chemical reactions and pathways resulting in the breakdown of elastin. Elastin is a glycoprotein which is randomly coiled and crosslinked to form elastic fibers that are found in connective tissue. Sources: GOC:BHF, GOC:dph, GOC:tb Also known as: elastin breakdown, elastin catabolism, elastin degradation